malate transport [GO:0015743] (biological process) Relationships: is a type of C4-dicarboxylate transport [GO:0015740] Subtypes: malic acid secretion [GO:0046723], malate transmembrane transport [GO:0071423] Definition: The directed movement of malate into, out of or within a cell, or between cells, by means of some agent such as a transporter or pore. Sources: GOC:krc Also known as: mitochondrial alpha-ketoglutarate/malate transport